{
  "term_id": "GO:0005730",
  "term_label": "nucleolus",
  "gene_symbol": "RRS1",
  "gene_name": "Ribosome biogenesis regulatory protein homolog",
  "gene": "UniProtKB:Q15050"
}